{
  "gene": "UniProtKB:Q9H903",
  "term_id": "GO:0004477",
  "term_label": "methenyltetrahydrofolate cyclohydrolase activity",
  "gene_name": "Bifunctional methylenetetrahydrofolate dehydrogenase_cyclohydrolase 2, mitochondrial",
  "gene_symbol": "MTHFD2L"
}